{
  "term_label": "regulation of circadian rhythm",
  "term_id": "GO:0042752",
  "gene": "UniProtKB:Q9UHM6",
  "gene_symbol": "OPN4",
  "gene_name": "Melanopsin"
}